positive regulation of male germ-line stem cell asymmetric division [GO:1904840] (biological process) Definition: Any process that activates or increases the frequency, rate or extent of male germ-line stem cell asymmetric division. References: PMID:19339709 Sources: GOC:TermGenie, GO_REF:0000058 Relationships: is a type of positive regulation of asymmetric cell division [GO:0045770]; is a type of positive regulation of multicellular organismal process [GO:0051240]; is a type of regulation of male germ-line stem cell asymmetric division [GO:1904838]; positively regulates GO:0048133 Also known as: positive regulation of male germ-line stem cell renewal, up regulation of male germ-line stem cell asymmetric division, up regulation of male germ-line stem cell renewal, up-regulation of male germ-line stem cell asymmetric division, up-regulation of male germ-line stem cell renewal, upregulation of male germ-line stem cell asymmetric division, upregulation of male germ-line stem cell renewal, activation of male germ-line stem cell asymmetric division, activation of male germ-line stem cell renewal